{
  "term_id": "UNKNOWN:0001",
  "gene_symbol": "TRBV20-1",
  "gene": "UniProtKB:A0A075B6N2",
  "term_label": "Unknown molecular function",
  "gene_name": "T cell receptor beta variable 20-1"
}